voltage-gated monoatomic ion channel activity involved in regulation of presynaptic membrane potential [GO:0099508] (molecular function) Definition: Voltage-gated ion channel activity, occurring in the presynaptic membrane, involved in regulation of presynaptic membrane potential. This is a key step in synaptic transmission, following the arrival of an action potential at the synapse. Sources: GOC:dos Also known as: voltage-gated ion channel activity involved in regulation of presynaptic membrane potential, voltage gated ion channel activity involved in regulation of presynaptic membrane potential, voltage-dependent ion channel activity involved in regulation of pre-synaptic membrane potential, voltage-dependent ion channel activity involved in regulation of presynaptic membrane potential, voltage-gated ion channel activity involved in regulation of pre-synaptic membrane potential Relationships: is a type of voltage-gated monoatomic ion channel activity [GO:0005244]; is part of regulation of presynaptic membrane potential [GO:0099505]; occurs in GO:0042734